IgG binding [GO:0019864] (molecular function) Definition: Binding to an immunoglobulin of an IgG isotype. Sources: GOC:add, ISBN:0781735149 Relationships: is a type of immunoglobulin binding [GO:0019865]